{
  "term_id": "GO:0046875",
  "gene": "UniProtKB:P98172",
  "term_label": "ephrin receptor binding",
  "gene_symbol": "EFNB1",
  "gene_name": "Ephrin-B1"
}